{
  "gene_name": "Neurofilament medium polypeptide",
  "gene": "UniProtKB:P07197",
  "term_id": "GO:0030424",
  "term_label": "axon",
  "gene_symbol": "NEFM"
}